primitive erythrocyte differentiation [GO:0060319] (biological process) Relationships: is_a erythrocyte differentiation [GO:0030218]; is part of GO:0060215 Sources: GOC:BHF, GOC:add, GOC:dph Definition: Erythrocyte differentiation which occurs as part of the process of primitive hemopoiesis. Regulation: regulated by GO:0010725 Also known as: primitive RBC differentiation, primitive erythropoiesis, primitive red blood cell differentiation